developmental pigmentation [GO:0048066] (biological process) Subtypes: cuticle pigmentation [GO:0048067], eye pigmentation [GO:0048069], sex-specific pigmentation [GO:0048071] Sources: ISBN:0582227089 Relationships: is a type of pigmentation [GO:0043473] Regulation: regulated by regulation of developmental pigmentation [GO:0048070]; negatively regulated by negative regulation of developmental pigmentation [GO:0048086]; positively regulated by positive regulation of developmental pigmentation [GO:0048087] Also known as: pigmentation during development Definition: The developmental process that results in the deposition of coloring matter in an organism, tissue or cell.